{
  "term_id": "GO:0016020",
  "term_label": "membrane",
  "gene_name": "Sialidase-3",
  "gene": "UniProtKB:Q9UQ49",
  "gene_symbol": "NEU3"
}